{
  "term_label": "rough endoplasmic reticulum",
  "gene_symbol": "HGFAC",
  "gene_name": "Hepatocyte growth factor activator",
  "gene": "UniProtKB:Q04756",
  "term_id": "GO:0005791"
}